{
  "gene_symbol": "OR5H15",
  "gene": "UniProtKB:A6NDH6",
  "gene_name": "Olfactory receptor 5H15",
  "term_label": "odorant binding",
  "term_id": "GO:0005549"
}